{
  "gene_name": "Monoacylglycerol_Diacylglycerol O-acyltransferase",
  "gene": "UniProtKB:Q96MH6",
  "term_label": "Unknown molecular function",
  "term_id": "UNKNOWN:0001",
  "gene_symbol": "TMEM68"
}